{
  "gene_symbol": "KLRC1",
  "term_label": "natural killer cell inhibitory signaling pathway",
  "term_id": "GO:0002769",
  "gene": "UniProtKB:P26715",
  "gene_name": "NKG2-A_NKG2-B type II integral membrane protein"
}